{
  "gene_symbol": "LETM2",
  "gene_name": "LETM1 domain-containing protein LETM2, mitochondrial",
  "term_id": "GO:0005739",
  "gene": "UniProtKB:Q2VYF4",
  "term_label": "mitochondrion"
}